{
  "term_id": "UNKNOWN:0001",
  "gene_name": "Golgin subfamily A member 6-like protein 6",
  "gene": "UniProtKB:A8MZA4",
  "term_label": "Unknown molecular function",
  "gene_symbol": "GOLGA6L6"
}